nitrogen catabolite activation of transcription from RNA polymerase II promoter [GO:0001080] (biological process) References: PMID:19104072 Sources: GOC:mah, GOC:txnOH Also known as: positive regulation of transcription from RNA polymerase II promoter by nitrogen catabolites Definition: A transcription regulation process in which the presence of one nitrogen source leads to an increase in the frequency, rate, or extent of transcription, from an RNA polymerase II promoter, of specific genes involved in the metabolism of other nitrogen sources. Relationships: is a type of nitrogen catabolite regulation of transcription from RNA polymerase II promoter [GO:0001079]; is a type of GO:0090294